{
  "term_label": "regulation of microtubule-based process",
  "gene_name": "Microtubule-actin cross-linking factor 1, isoforms 1_2_3_4_5",
  "gene_symbol": "MACF1",
  "term_id": "GO:0032886",
  "gene": "UniProtKB:Q9UPN3"
}